{
  "gene_symbol": "SLC6A11",
  "term_id": "GO:0042995",
  "term_label": "cell projection",
  "gene": "UniProtKB:P48066",
  "gene_name": "Sodium- and chloride-dependent GABA transporter 3"
}